{
  "term_label": "intermediate filament organization",
  "gene_name": "Keratin, type I cytoskeletal 15",
  "gene": "UniProtKB:P19012",
  "term_id": "GO:0045109",
  "gene_symbol": "KRT15"
}